{
  "gene_symbol": "AP1M2",
  "term_id": "GO:0030121",
  "term_label": "AP-1 adaptor complex",
  "gene_name": "AP-1 complex subunit mu-2",
  "gene": "UniProtKB:Q9Y6Q5"
}